{
  "gene": "UniProtKB:P40200",
  "term_label": "cell-matrix adhesion",
  "gene_name": "T-cell surface protein tactile",
  "gene_symbol": "CD96",
  "term_id": "GO:0007160"
}